structural constituent of chitin-based larval cuticle [GO:0008010] (molecular function) Sources: GOC:mah, GOC:mtg_sensu Definition: The action of a molecule that contributes to the structural integrity of the chitin-based cuticle of a larva. An example of this is found in Drosophila melanogaster. Relationships: is a type of structural constituent of chitin-based cuticle [GO:0005214] Also known as: structural constituent of larval cuticle